{
  "term_label": "ferric iron binding",
  "term_id": "GO:0008199",
  "gene_symbol": "FXN",
  "gene": "UniProtKB:Q16595",
  "gene_name": "Frataxin, mitochondrial"
}